{
  "gene": "UniProtKB:O76013",
  "term_label": "cytoskeleton",
  "gene_name": "Keratin, type I cuticular Ha6",
  "term_id": "GO:0005856",
  "gene_symbol": "KRT36"
}